negative regulation of prostaglandin catabolic process [GO:1905829] (biological process) Also known as: down regulation of prostaglandin breakdown, down regulation of prostaglandin catabolic process, down regulation of prostaglandin catabolism, down regulation of prostaglandin degradation, down-regulation of prostaglandin breakdown, down-regulation of prostaglandin catabolic process, down-regulation of prostaglandin catabolism, down-regulation of prostaglandin degradation, downregulation of prostaglandin breakdown, downregulation of prostaglandin catabolic process, downregulation of prostaglandin catabolism, downregulation of prostaglandin degradation, negative regulation of prostaglandin breakdown, negative regulation of prostaglandin catabolism, negative regulation of prostaglandin degradation, inhibition of prostaglandin breakdown, inhibition of prostaglandin catabolic process, inhibition of prostaglandin catabolism, inhibition of prostaglandin degradation Relationships: is a type of negative regulation of lipid catabolic process [GO:0050995]; is a type of regulation of prostaglandin catabolic process [GO:1905828]; negatively regulates prostaglandin catabolic process [GO:1905344] Definition: Any process that stops, prevents or reduces the frequency, rate or extent of prostaglandin catabolic process. References: PMID:12432938 Sources: GOC:TermGenie, GO_REF:0000058